{
  "gene_symbol": "OPHN1",
  "gene_name": "Oligophrenin-1",
  "gene": "UniProtKB:O60890",
  "term_id": "GO:0043195",
  "term_label": "terminal bouton"
}